negative regulation of metanephric glomerular mesangial cell proliferation [GO:0072302] (biological process) Relationships: is a type of GO:0072125; is a type of regulation of metanephric glomerular mesangial cell proliferation [GO:0072301]; negatively regulates GO:0072262 Sources: GOC:mtg_kidney_jan10 Definition: Any process that decreases the frequency, rate or extent of metanephric glomerular mesangial cell proliferation.